{
  "gene": "UniProtKB:Q6ZN11",
  "gene_symbol": "ZNF793",
  "term_label": "regulation of transcription by RNA polymerase II",
  "gene_name": "Zinc finger protein 793",
  "term_id": "GO:0006357"
}